{
  "term_label": "IPAF inflammasome complex",
  "gene": "UniProtKB:P29466",
  "term_id": "GO:0072557",
  "gene_name": "Caspase-1",
  "gene_symbol": "CASP1"
}